{
  "gene_symbol": "MBP",
  "gene": "UniProtKB:P02686",
  "term_label": "cell periphery",
  "term_id": "GO:0071944",
  "gene_name": "Myelin basic protein"
}